{
  "term_id": "GO:0004896",
  "gene_name": "Tissue factor",
  "term_label": "cytokine receptor activity",
  "gene_symbol": "F3",
  "gene": "UniProtKB:P13726"
}